{
  "term_label": "basic amino acid transmembrane transporter activity",
  "gene": "UniProtKB:Q9UM01",
  "term_id": "GO:0015174",
  "gene_symbol": "SLC7A7",
  "gene_name": "Y+L amino acid transporter 1"
}